{
  "gene": "UniProtKB:Q96E11",
  "gene_name": "Ribosome-recycling factor, mitochondrial",
  "gene_symbol": "MRRF",
  "term_id": "GO:0043023",
  "term_label": "ribosomal large subunit binding"
}